translation at synapse [GO:0140241] (biological process) Note: Note that this term was created for the SynGO project, and will be obsoleted when the SynGO annotations are made in Noctua. Relationships: is a type of translation [GO:0006412]; occurs in synapse [GO:0045202] Definition: Translation that occurs at the synapse. Subtypes: translation at presynapse [GO:0140236], translation at postsynapse [GO:0140242] References: PMID:23083742